{
  "gene": "UniProtKB:Q99618",
  "term_id": "UNKNOWN:0002",
  "term_label": "Unknown biological process",
  "gene_symbol": "CDCA3",
  "gene_name": "Cell division cycle-associated protein 3"
}